negative regulation of collateral sprouting of intact axon in response to injury [GO:0048685] (biological process) Relationships: is a type of GO:0048671; is a type of negative regulation of axon regeneration [GO:0048681]; is a type of GO:0048683; negatively regulates collateral sprouting of intact axon in response to injury [GO:0048673] Also known as: down regulation of collateral sprouting of intact axon in response to injury, down-regulation of collateral sprouting of intact axon in response to injury, downregulation of collateral sprouting of intact axon in response to injury, inhibition of collateral sprouting of intact axon in response to injury Definition: Any process that stops, prevents, or reduces the frequency, rate or extent of collateral sprouting of an intact axon as a result of injury to an axon. Sources: GOC:dgh, GOC:dph, GOC:jid, GOC:lm